hydroxyproline O-arabinosyltransferase activity [GO:1990585] (molecular function) Definition: Catalysis of the reaction: trans-4-hydroxy-L-prolyl-[protein] + UDP-beta-L-arabinofuranose = H+ + O-(beta-L-arabinofuranosyl)-trans-4-hydroxy-L-prolyl-[protein] + UDP. Also known as: HPAT Relationships: is a type of pentosyltransferase activity [GO:0016763] References: PMID:24036508 Sources: RHEA:49472